positive regulation of serotonin secretion [GO:0014064] (BP) Definition: Any process that activates or increases the frequency, rate or extent of the regulated release of serotonin. Sources: GOC:ef Also known as: up regulation of serotonin secretion, up-regulation of serotonin secretion, upregulation of serotonin secretion, activation of serotonin secretion, stimulation of serotonin secretion, positive regulation of serotonin release Relationships: is a type of GO:0014062; is a type of positive regulation of monoatomic ion transport [GO:0043270]; is a type of positive regulation of secretion by cell [GO:1903532]; positively regulates serotonin secretion [GO:0001820]